{
  "term_label": "histone deacetylase complex",
  "term_id": "GO:0000118",
  "gene_name": "PHD finger protein 21A",
  "gene": "UniProtKB:Q96BD5",
  "gene_symbol": "PHF21A"
}